G-rich strand telomeric DNA binding [GO:0098505] (molecular function) Relationships: is a type of single-stranded telomeric DNA binding [GO:0043047] Definition: Binding to G-rich, single-stranded, telomere-associated DNA. References: PMID:11349150